{
  "term_id": "GO:0000978",
  "term_label": "RNA polymerase II cis-regulatory region sequence-specific DNA binding",
  "gene_name": "Zinc finger protein 524",
  "gene": "UniProtKB:Q96C55",
  "gene_symbol": "ZNF524"
}